{
  "term_label": "L-proline catabolic process",
  "gene_name": "D-amino-acid oxidase",
  "gene": "UniProtKB:P14920",
  "gene_symbol": "DAO",
  "term_id": "GO:0006562"
}